{
  "gene": "UniProtKB:P56202",
  "term_label": "cysteine-type endopeptidase activity",
  "gene_name": "Cathepsin W",
  "gene_symbol": "CTSW",
  "term_id": "GO:0004197"
}